coniferin beta-glucosidase activity [GO:0047782] (molecular function) Definition: Catalysis of the reaction: H2O + coniferin = D-glucose + coniferol. Sources: EC:3.2.1.126, MetaCyc:CONIFERIN-BETA-GLUCOSIDASE-RXN Also known as: coniferin b-glucosidase activity, coniferin beta-D-glucosidase activity, coniferin-hydrolyzing beta-glucosidase activity Relationships: is a type of beta-glucosidase activity [GO:0008422]